{
  "gene_symbol": "NR2C2AP",
  "gene_name": "Nuclear receptor 2C2-associated protein",
  "term_id": "UNKNOWN:0003",
  "gene": "UniProtKB:Q86WQ0",
  "term_label": "Unknown cellular component"
}